{
  "gene": "UniProtKB:Q8NH72",
  "term_label": "plasma membrane",
  "gene_symbol": "OR4C6",
  "gene_name": "Olfactory receptor 4C6",
  "term_id": "GO:0005886"
}